{
  "term_id": "GO:0000978",
  "gene_name": "Hairy_enhancer-of-split related with YRPW motif protein 1",
  "gene_symbol": "HEY1",
  "gene": "UniProtKB:Q9Y5J3",
  "term_label": "RNA polymerase II cis-regulatory region sequence-specific DNA binding"
}